cochlear nucleus development [GO:0021747] (biological process) Sources: GOC:cls, GOC:curators, GOC:dgh, GOC:dph, GOC:jid Subtypes: dorsal cochlear nucleus development [GO:0021748], ventral cochlear nucleus development [GO:0021749] Relationships: is a type of neural nucleus development [GO:0048857]; is part of pons development [GO:0021548] Definition: The process whose specific outcome is the progression of the cochlear nucleus over time, from its formation to the mature structure.